{
  "term_label": "cytoplasm",
  "gene_symbol": "MAP3K10",
  "gene": "UniProtKB:Q02779",
  "term_id": "GO:0005737",
  "gene_name": "Mitogen-activated protein kinase kinase kinase 10"
}